{
  "gene": "UniProtKB:Q9H9J4",
  "gene_name": "Ubiquitin carboxyl-terminal hydrolase 42",
  "gene_symbol": "USP42",
  "term_id": "GO:0004843",
  "term_label": "cysteine-type deubiquitinase activity"
}